{
  "gene_name": "Vang-like protein 2",
  "gene_symbol": "VANGL2",
  "term_label": "establishment of planar polarity",
  "gene": "UniProtKB:Q9ULK5",
  "term_id": "GO:0001736"
}